{
  "gene_symbol": "INTS10",
  "gene": "UniProtKB:Q9NVR2",
  "term_id": "GO:0032039",
  "gene_name": "Integrator complex subunit 10",
  "term_label": "integrator complex"
}